{
  "term_id": "GO:0042391",
  "gene_name": "Potassium voltage-gated channel subfamily H member 1",
  "gene": "UniProtKB:O95259",
  "gene_symbol": "KCNH1",
  "term_label": "regulation of membrane potential"
}